{
  "term_label": "DNA binding",
  "gene_symbol": "H2BC11",
  "term_id": "GO:0003677",
  "gene": "UniProtKB:P06899",
  "gene_name": "Histone H2B type 1-J"
}